{
  "gene_symbol": "CDK8",
  "gene_name": "Cyclin-dependent kinase 8",
  "term_label": "cyclin-dependent protein serine/threonine kinase activity",
  "term_id": "GO:0004693",
  "gene": "UniProtKB:P49336"
}